Noc2p-Noc3p complex [GO:0030691] (cellular component) Note: Noc complexes exhibit a dynamic intranuclear location; consider also annotating to 'nucleolus ; GO:0005730' and/or 'nucleoplasm ; GO:0005654'. Note that the term name uses Saccharomyces gene product names because no other names have yet arisen for this complex; the term nevertheless can be used for analogous complexes in other eukaryotes, and the name can be changed if better wording is found. Definition: A heterodimer associated with 66S preribosomes; predominantly nucleoplasmic, but also locates to the nucleolus; involved in ribosomal large subunit biogenesis. Relationships: is a type of Noc complex [GO:0030689]; is part of GO:0030687 References: PMID:12446671